{
  "gene_name": "Glycosyltransferase 8 domain-containing protein 2",
  "gene": "UniProtKB:Q9H1C3",
  "term_label": "Golgi apparatus",
  "gene_symbol": "GLT8D2",
  "term_id": "GO:0005794"
}